{
  "gene_symbol": "PABPC1L2A",
  "gene_name": "Polyadenylate-binding protein 1-like 2",
  "term_id": "GO:0003730",
  "gene": "UniProtKB:Q5JQF8",
  "term_label": "mRNA 3'-UTR binding"
}